{
  "term_label": "Unknown molecular function",
  "term_id": "UNKNOWN:0001",
  "gene_symbol": "KRTAP10-1",
  "gene_name": "Keratin-associated protein 10-1",
  "gene": "UniProtKB:P60331"
}